TFIIIC-TOP1-SUB1 complex [GO:0034740] (cellular component) Definition: A protein complex that contains TFIIIC, topoisomerase 1, and Sub1/PC4. Characterized in human, the complex is involved in regulating transcription from RNA polymerase III (Pol III) promoters. Topoisomerase 1 and Sub1 enhance the accuracy of transcription termination, and promote reinitiation by Pol III. References: PMID:9660958 Also known as: TFIIIC-Topoisomerase 1-PC4 complex Relationships: is a type of RNA polymerase III transcription regulator complex [GO:0090576]